{
  "gene": "UniProtKB:P32243",
  "term_id": "GO:0005634",
  "gene_symbol": "OTX2",
  "gene_name": "Homeobox protein OTX2",
  "term_label": "nucleus"
}